histone H2AR3 methyltransferase activity [GO:0070612] (molecular function) References: PMID:17898714, PMID:23451136 Sources: GOC:mah Definition: Catalysis of the reaction: S-adenosyl-L-methionine + (histone H2A)-arginine (position 3) = S-adenosyl-L-homocysteine + (histone H2A)-N-methyl-arginine (position 3). This reaction is the addition of a methyl group to the arginine residue at position 3 of histone H2A. Relationships: is a type of GO:0016274; is a type of histone H2A methyltransferase activity [GO:0140940] Note: Note that the residue position corresponds to the canonical human H2A2A histone (UniProtKB:Q6FI13); this residue seems to be only present in animals. Residue 1 is the first residue following removal of the initiating Methionine (Met). Note that each histone is encoded by multiple genes, and sequences may vary across different genes within an organism. Also known as: histone H2AR3 arginine methyltransferase activity, histone methylase activity (H2A-R3 specific), histone methyltransferase activity (H2A-R3 specific), histone-H2AR3 methyltransferase activity, histone-arginine N-methyltransferase activity (H2A-R3 specific)